{
  "term_label": "fertilization",
  "term_id": "GO:0009566",
  "gene_name": "RIMS-binding protein 3B",
  "gene_symbol": "RIMBP3B",
  "gene": "UniProtKB:A6NNM3"
}